detection of cAMP [GO:0031319] (biological process) Sources: GOC:pg Relationships: is a type of detection of chemical stimulus [GO:0009593]; is a type of GO:0051591 Also known as: 3',5'-cAMP detection, 3',5'-cAMP sensing, cAMP detection, cAMP sensing, cyclic AMP detection, detection of 3',5' cAMP, detection of 3',5'-cAMP, detection of adenosine 3',5'-cyclophosphate, detection of cyclic AMP Definition: The series of events in which a cAMP (cyclic AMP, adenosine 3',5'-cyclophosphate) stimulus is received by a cell and converted into a molecular signal; cAMP is the nucleotide cyclic AMP.